{
  "term_id": "GO:0007165",
  "gene_symbol": "GAB4",
  "gene": "UniProtKB:Q2WGN9",
  "gene_name": "GRB2-associated-binding protein 4",
  "term_label": "signal transduction"
}